{
  "term_label": "Unknown biological process",
  "gene_name": "Golgin subfamily A member 6-like protein 1",
  "gene": "UniProtKB:Q8N7Z2",
  "term_id": "UNKNOWN:0002",
  "gene_symbol": "GOLGA6L1"
}